{
  "gene_name": "MOB kinase activator 3C",
  "term_label": "protein kinase activator activity",
  "term_id": "GO:0030295",
  "gene_symbol": "MOB3C",
  "gene": "UniProtKB:Q70IA8"
}